{
  "gene": "UniProtKB:Q9NR90",
  "term_label": "cytoplasm",
  "gene_symbol": "DAZ3",
  "term_id": "GO:0005737",
  "gene_name": "Deleted in azoospermia protein 3"
}